positive regulation of kojic acid biosynthetic process [GO:1900396] (biological process) Relationships: is a type of regulation of kojic acid biosynthetic process [GO:1900394]; is a type of GO:1902932; RO_0002213 kojic acid biosynthetic process [GO:2001317] Definition: Any process that activates or increases the frequency, rate or extent of kojic acid biosynthetic process. Also known as: activation of 5-hydroxy-2-(hydroxymethyl)-4H-pyran-4-one anabolism, activation of 5-hydroxy-2-(hydroxymethyl)-4H-pyran-4-one biosynthesis, activation of 5-hydroxy-2-(hydroxymethyl)-4H-pyran-4-one biosynthetic process, activation of 5-hydroxy-2-(hydroxymethyl)-4H-pyran-4-one formation, activation of 5-hydroxy-2-(hydroxymethyl)-4H-pyran-4-one synthesis, activation of kojic acid anabolism, activation of kojic acid biosynthesis, activation of kojic acid formation, activation of kojic acid synthesis, positive regulation of 5-hydroxy-2-(hydroxymethyl)-4H-pyran-4-one anabolism, positive regulation of 5-hydroxy-2-(hydroxymethyl)-4H-pyran-4-one biosynthesis, positive regulation of 5-hydroxy-2-(hydroxymethyl)-4H-pyran-4-one biosynthetic process, positive regulation of 5-hydroxy-2-(hydroxymethyl)-4H-pyran-4-one formation, positive regulation of 5-hydroxy-2-(hydroxymethyl)-4H-pyran-4-one synthesis, positive regulation of kojic acid anabolism, positive regulation of kojic acid biosynthesis, positive regulation of kojic acid formation, positive regulation of kojic acid synthesis, up regulation of 5-hydroxy-2-(hydroxymethyl)-4H-pyran-4-one anabolism, up regulation of 5-hydroxy-2-(hydroxymethyl)-4H-pyran-4-one biosynthesis, up regulation of 5-hydroxy-2-(hydroxymethyl)-4H-pyran-4-one biosynthetic process, up regulation of 5-hydroxy-2-(hydroxymethyl)-4H-pyran-4-one formation, up regulation of 5-hydroxy-2-(hydroxymethyl)-4H-pyran-4-one synthesis, up regulation of kojic acid anabolism, up regulation of kojic acid biosynthesis, up regulation of kojic acid biosynthetic process, up regulation of kojic acid formation, up regulation of kojic acid synthesis, up-regulation of 5-hydroxy-2-(hydroxymethyl)-4H-pyran-4-one anabolism, up-regulation of 5-hydroxy-2-(hydroxymethyl)-4H-pyran-4-one biosynthesis, up-regulation of 5-hydroxy-2-(hydroxymethyl)-4H-pyran-4-one biosynthetic process, up-regulation of 5-hydroxy-2-(hydroxymethyl)-4H-pyran-4-one formation, up-regulation of 5-hydroxy-2-(hydroxymethyl)-4H-pyran-4-one synthesis, up-regulation of kojic acid anabolism, up-regulation of kojic acid biosynthesis, up-regulation of kojic acid biosynthetic process, up-regulation of kojic acid formation, up-regulation of kojic acid synthesis, upregulation of 5-hydroxy-2-(hydroxymethyl)-4H-pyran-4-one anabolism, upregulation of 5-hydroxy-2-(hydroxymethyl)-4H-pyran-4-one biosynthesis, upregulation of 5-hydroxy-2-(hydroxymethyl)-4H-pyran-4-one biosynthetic process, upregulation of 5-hydroxy-2-(hydroxymethyl)-4H-pyran-4-one formation, upregulation of 5-hydroxy-2-(hydroxymethyl)-4H-pyran-4-one synthesis, upregulation of kojic acid anabolism, upregulation of kojic acid biosynthesis, upregulation of kojic acid biosynthetic process, upregulation of kojic acid formation, upregulation of kojic acid synthesis, activation of kojic acid biosynthetic process, activation of C6H6O4 anabolism, activation of C6H6O4 biosynthesis, activation of C6H6O4 biosynthetic process, activation of C6H6O4 formation, activation of C6H6O4 synthesis, positive regulation of C6H6O4 anabolism, positive regulation of C6H6O4 biosynthesis, positive regulation of C6H6O4 biosynthetic process, positive regulation of C6H6O4 formation, positive regulation of C6H6O4 synthesis, up regulation of C6H6O4 anabolism, up regulation of C6H6O4 biosynthesis, up regulation of C6H6O4 biosynthetic process, up regulation of C6H6O4 formation, up regulation of C6H6O4 synthesis, up-regulation of C6H6O4 anabolism, up-regulation of C6H6O4 biosynthesis, up-regulation of C6H6O4 biosynthetic process, up-regulation of C6H6O4 formation, up-regulation of C6H6O4 synthesis, upregulation of C6H6O4 anabolism, upregulation of C6H6O4 biosynthesis, upregulation of C6H6O4 biosynthetic process, upregulation of C6H6O4 formation, upregulation of C6H6O4 synthesis Sources: GOC:TermGenie, GOC:di